{
  "gene_symbol": "CHRNA10",
  "term_label": "plasma membrane",
  "term_id": "GO:0005886",
  "gene_name": "Neuronal acetylcholine receptor subunit alpha-10",
  "gene": "UniProtKB:Q9GZZ6"
}